class II DNA-(apurinic or apyrimidinic site) endonuclease activity [GO:0052720] (molecular function) Definition: Catalysis of the hydrolysis of ester linkages immediately 5' to an apurinic/apyrimidinic (AP; also called abasic) site within a deoxyribonucleic acid molecule by creating internal breaks, generating a single-strand break with 5'-deoxyribose phosphate and 3'-hydroxyl ends. Also known as: class II DNA-(apurinic or apyrimidinic site) lyase activity, class II AP endonuclease activity References: PMID:1698278 Relationships: is a type of DNA-(apurinic or apyrimidinic site) endonuclease activity [GO:0003906]; is_a DNA endonuclease activity, producing 5'-phosphomonoesters [GO:0016888]